{
  "gene_symbol": "PFN1",
  "gene": "UniProtKB:P07737",
  "gene_name": "Profilin-1",
  "term_label": "cytoplasm",
  "term_id": "GO:0005737"
}